{
  "gene_symbol": "ACOX3",
  "term_label": "flavin adenine dinucleotide binding",
  "term_id": "GO:0050660",
  "gene_name": "Peroxisomal acyl-coenzyme A oxidase 3",
  "gene": "UniProtKB:O15254"
}